cis-2,3-dihydrobiphenyl-2,3-diol dehydrogenase activity [GO:0018509] (MF) Relationships: is a type of GO:0016628 Also known as: 2,3-dihydro-2,3-dihydroxybiphenyl dehydrogenase activity, biphenyl-2,3-dihydro-2,3-diol dehydrogenase activity, cis-3-phenylcyclohexa-3,5-diene-1,2-diol:NAD+ oxidoreductase activity Definition: Catalysis of the reaction: cis-3-phenylcyclohexa-3,5-diene-1,2-diol + NAD+ = biphenyl-2,3-diol + NADH + H+. Sources: EC:1.3.1.56